{
  "term_id": "GO:0001822",
  "gene": "UniProtKB:Q13099",
  "gene_name": "Intraflagellar transport protein 88 homolog",
  "gene_symbol": "IFT88",
  "term_label": "kidney development"
}